methionine adenosyltransferase regulator activity [GO:0048270] (molecular function) Definition: Binds to and modulates the activity of methionine adenosyltransferase. Also known as: MAT regulator activity Relationships: is_a enzyme regulator activity [GO:0030234]; regulates methionine adenosyltransferase activity [GO:0004478] References: PMID:10644686 Sources: GOC:jid Note: See also the molecular function term 'methionine adenosyltransferase activity ; GO:0004478'.